{
  "gene_name": "Lysophosphatidic acid receptor 3",
  "gene_symbol": "LPAR3",
  "gene": "UniProtKB:Q9UBY5",
  "term_id": "GO:0005737",
  "term_label": "cytoplasm"
}